{
  "gene": "UniProtKB:Q05193",
  "gene_name": "Dynamin-1",
  "term_label": "synaptic vesicle budding from presynaptic endocytic zone membrane",
  "term_id": "GO:0016185",
  "gene_symbol": "DNM1"
}